{
  "gene_symbol": "CERS5",
  "term_label": "sphingosine N-acyltransferase activity",
  "gene": "UniProtKB:Q8N5B7",
  "gene_name": "Ceramide synthase 5",
  "term_id": "GO:0050291"
}